{
  "term_label": "vitamin D metabolic process",
  "gene_symbol": "GC",
  "term_id": "GO:0042359",
  "gene_name": "Vitamin D-binding protein",
  "gene": "UniProtKB:P02774"
}